{
  "gene_name": "SWI_SNF-related matrix-associated actin-dependent regulator of chromatin subfamily E member 1-related",
  "term_label": "regulation of gene expression",
  "gene_symbol": "HMG20B",
  "gene": "UniProtKB:Q9P0W2",
  "term_id": "GO:0010468"
}